negative regulation of receptor recycling [GO:0001920] (biological process) Definition: Any process that stops, prevents, or reduces the rate of receptor recycling. Sources: GOC:add Also known as: down regulation of receptor recycling, down-regulation of receptor recycling, downregulation of receptor recycling, inhibition of receptor recycling Relationships: is a type of regulation of receptor recycling [GO:0001919]; is a type of GO:0010605; is a type of negative regulation of signaling [GO:0023057]; negatively regulates receptor recycling [GO:0001881]